{
  "term_id": "GO:0035567",
  "gene": "UniProtKB:O75084",
  "gene_name": "Frizzled-7",
  "term_label": "non-canonical Wnt signaling pathway",
  "gene_symbol": "FZD7"
}